{
  "gene_name": "Exocyst complex component 4",
  "term_id": "GO:0007268",
  "gene_symbol": "EXOC4",
  "term_label": "chemical synaptic transmission",
  "gene": "UniProtKB:Q96A65"
}